{
  "term_id": "GO:0005634",
  "gene_name": "Proteasome subunit beta type-6",
  "term_label": "nucleus",
  "gene_symbol": "PSMB6",
  "gene": "UniProtKB:P28072"
}